{
  "gene_symbol": "STMND1",
  "gene_name": "Stathmin domain-containing protein 1",
  "term_label": "neuron projection development",
  "term_id": "GO:0031175",
  "gene": "UniProtKB:H3BQB6"
}